{
  "gene": "UniProtKB:Q15072",
  "term_label": "RNA polymerase II cis-regulatory region sequence-specific DNA binding",
  "term_id": "GO:0000978",
  "gene_name": "Zinc finger protein OZF",
  "gene_symbol": "ZNF146"
}